gibberellin beta-D-glucosyltransferase activity [GO:0047928] (molecular function) Also known as: gibberellin b-glucosyltransferase activity, UDP-glucose:gibberellin 2-O-beta-D-glucosyltransferase activity, UDPglucose:gibberellin 2-O-beta-D-glucosyltransferase activity, uridine diphosphoglucose-gibberellate 3-O-glucosyltransferase activity, uridine diphosphoglucose-gibberellate 7-glucosyltransferase activity Relationships: is a type of UDP-glucosyltransferase activity [GO:0035251] Definition: Catalysis of the reaction: UDP-glucose + gibberellin = UDP + gibberellin 2-O-beta-D-glucoside. Sources: EC:2.4.1.176, MetaCyc:GIBBERELLIN-BETA-GLUCOSYLTRANSFERASE-RXN